{
  "term_label": "Unknown biological process",
  "gene_name": "Piercer of microtubule wall 2 protein",
  "term_id": "UNKNOWN:0002",
  "gene_symbol": "PIERCE2",
  "gene": "UniProtKB:H3BRN8"
}